regulation of cytoskeleton organization [GO:0051493] (biological process) Subtypes: regulation of cytoskeleton polarization involved in growth plate cartilage chondrocyte division [GO:0003427], regulation of actin cytoskeleton organization [GO:0032956], negative regulation of cytoskeleton organization [GO:0051494], positive regulation of cytoskeleton organization [GO:0051495], regulation of pseudohyphal septin ring assembly [GO:0062164], GO:0070507 Relationships: is a type of regulation of organelle organization [GO:0033043]; RO_0002211 cytoskeleton organization [GO:0007010] Definition: Any process that modulates the frequency, rate or extent of the formation, arrangement of constituent parts, or disassembly of cytoskeletal structures. Also known as: regulation of cytoskeleton organisation, regulation of cytoskeleton organization and biogenesis Sources: GOC:ai